glyoxysomal lumen [GO:0031908] (cellular component) Definition: The volume enclosed by the membranes of a glyoxysome. Relationships: is a type of GO:0005782 Sources: GOC:mah